{
  "term_id": "GO:0006357",
  "gene_name": "Zinc finger and SCAN domain-containing protein 26",
  "term_label": "regulation of transcription by RNA polymerase II",
  "gene": "UniProtKB:Q16670",
  "gene_symbol": "ZSCAN26"
}